dolichyl pyrophosphate Glc1Man9GlcNAc2 alpha-1,3-glucosyltransferase activity [GO:0042283] (molecular function) References: PMID:12480927 Sources: MetaCyc:RXN-5471 Relationships: is a type of dolichyl-phosphate-glucose-glycolipid alpha-glucosyltransferase activity [GO:0004583] Also known as: dolichyl-P-Glc:Glc1Man9GlcNAc2-PP-dolichyl glucosyltransferase activity Definition: Catalysis of the addition of the second glucose residue to the lipid-linked oligosaccharide precursor for N-linked glycosylation; the transfer of glucose from dolichyl phosphate glucose (Dol-P-Glc) on to the lipid-linked oligosaccharide Glc(1)Man(9)GlcNAc(2)-PP-Dol.